positive regulation of cellulose catabolic process [GO:2000999] (biological process) Relationships: is a type of positive regulation of catabolic process [GO:0009896]; is_a positive regulation of macromolecule metabolic process [GO:0010604]; is a type of positive regulation of carbohydrate metabolic process [GO:0045913]; is a type of regulation of cellulose catabolic process [GO:2000997]; positively regulates cellulose catabolic process [GO:0030245] Also known as: positive regulation of cellulose breakdown, positive regulation of cellulose catabolism, positive regulation of cellulose degradation Sources: GOC:mengo_curators Definition: Any process that activates or increases the frequency, rate or extent of cellulose catabolic process.